insulin-like growth factor II binding [GO:0031995] (molecular function) Also known as: IGF-II binding Relationships: is a type of GO:0005520 Sources: GOC:mah Definition: Binding to insulin-like growth factor II.